external side of apical plasma membrane [GO:0098591] (CC) Definition: The leaflet the apical region of the plasma membrane that faces away from the cytoplasm and any proteins embedded or anchored in it or attached to its surface. Sources: GOC:ab, GOC:dos Relationships: is a type of external side of plasma membrane [GO:0009897]; is part of apical plasma membrane [GO:0016324]